{
  "gene_name": "ATP-dependent RNA helicase A",
  "term_label": "regulation of mRNA processing",
  "term_id": "GO:0050684",
  "gene_symbol": "DHX9",
  "gene": "UniProtKB:Q08211"
}